optic cup formation involved in camera-type eye development [GO:0003408] (biological process) Definition: The developmental process pertaining to the initial formation of the optic cup, a two-walled vesicle formed from the optic vesicle. Relationships: is_a anatomical structure formation involved in morphogenesis [GO:0048646]; is part of optic cup morphogenesis involved in camera-type eye development [GO:0002072] Sources: GOC:ascb_2009, GOC:dph, GOC:tb